{
  "gene_name": "Translation machinery-associated protein 7B",
  "gene": "UniProtKB:A0A024R1R8",
  "term_label": "Unknown molecular function",
  "term_id": "UNKNOWN:0001",
  "gene_symbol": "TMA7B"
}